{
  "term_id": "GO:0001518",
  "gene_name": "Sodium channel subunit beta-3",
  "term_label": "voltage-gated sodium channel complex",
  "gene": "UniProtKB:Q9NY72",
  "gene_symbol": "SCN3B"
}